{
  "gene": "UniProtKB:Q86UQ0",
  "gene_symbol": "ZNF589",
  "term_label": "RNA polymerase II cis-regulatory region sequence-specific DNA binding",
  "term_id": "GO:0000978",
  "gene_name": "Zinc finger protein 589"
}